negative regulation of reciprocal meiotic recombination [GO:0045128] (biological process) Definition: Any process that decreases the frequency, rate or extent of recombination during meiosis. Reciprocal meiotic recombination is the cell cycle process in which double strand breaks are formed and repaired through a double Holliday junction intermediate. Sources: GOC:ai, GOC:dph, GOC:tb Also known as: down regulation of meiotic recombination, down-regulation of meiotic recombination, downregulation of meiotic recombination, suppression of meiotic recombination, inhibition of meiotic recombination Relationships: is_a regulation of reciprocal meiotic recombination [GO:0010520]; is a type of negative regulation of meiotic nuclear division [GO:0045835]; is a type of negative regulation of DNA recombination [GO:0045910]; negatively regulates GO:0007131